{
  "gene_name": "Suppressor of cytokine signaling 2",
  "gene": "UniProtKB:O14508",
  "term_id": "UNKNOWN:0003",
  "gene_symbol": "SOCS2",
  "term_label": "Unknown cellular component"
}